{
  "gene": "UniProtKB:O95832",
  "gene_symbol": "CLDN1",
  "gene_name": "Claudin-1",
  "term_id": "GO:0005923",
  "term_label": "bicellular tight junction"
}